{
  "gene_name": "Cadherin-11",
  "gene": "UniProtKB:P55287",
  "gene_symbol": "CDH11",
  "term_id": "GO:0045296",
  "term_label": "cadherin binding"
}